5'-(N(7)-methylguanosine 5'-triphospho)-[mRNA] hydrolase activity [GO:0140933] (molecular function) Also known as: m(7)GpppN-mRNA hydrolase activity Definition: Catalysis of the reaction: a 5'-end (N7-methyl 5'-triphosphoguanosine)-ribonucleoside in mRNA + H2O = a 5'-end phospho-ribonucleoside in mRNA + N7-methyl-GDP + H+. References: PMID:18820299, PMID:29483298 Relationships: is a type of GO:0016462